2-aminobenzenesulfonate catabolic process [GO:0046230] (biological process) Subtypes: 2-aminobenzenesulfonate desulfonation [GO:0019490] Relationships: is a type of GO:0009310; is a type of organic acid catabolic process [GO:0016054]; is a type of xenobiotic catabolic process [GO:0042178]; is a type of benzene-containing compound metabolic process [GO:0042537]; is a type of sulfur compound catabolic process [GO:0044273] Definition: The chemical reactions and pathways resulting in the breakdown of 2-aminobenzenesulfonate, an aromatic sulfonate used in organic synthesis and in the manufacture of various dyes and medicines. Also known as: 2-aminobenzenesulfonate breakdown, 2-aminobenzenesulfonate catabolism, 2-aminobenzenesulfonate degradation, 2-aminobenzenesulphonate catabolic process, 2-aminobenzenesulphonate catabolism Sources: GOC:ai